amidophosphoribosyltransferase activity [GO:0004044] (MF) Sources: EC:2.4.2.14, RHEA:14905 Also known as: 5'-phosphoribosylpyrophosphate amidotransferase activity, 5-phosphoribosyl-1-pyrophosphate amidotransferase activity, 5-phosphoribosylamine:diphosphate phospho-alpha-D-ribosyltransferase (glutamate-amidating), 5-phosphororibosyl-1-pyrophosphate amidotransferase activity, alpha-5-phosphoribosyl-1-pyrophosphate amidotransferase activity, glutamine 5-phosphoribosylpyrophosphate amidotransferase activity, glutamine phosphoribosyldiphosphate amidotransferase activity, glutamine phosphoribosylpyrophosphate amidotransferase activity, glutamine ribosylpyrophosphate 5-phosphate amidotransferase activity, phosphoribose pyrophosphate amidotransferase activity, phosphoribosyl pyrophosphate amidotransferase activity, phosphoribosyldiphosphate 5-amidotransferase activity, phosphoribosylpyrophosphate glutamyl amidotransferase activity Definition: Catalysis of the reaction: 5-phospho-beta-D-ribosylamine + L-glutamate + diphosphate = 5-phospho-alpha-D-ribose 1-diphosphate + L-glutamine + H2O. Relationships: is_a GO:0016763